{
  "term_id": "UNKNOWN:0003",
  "term_label": "Unknown cellular component",
  "gene_symbol": "TMEM9B",
  "gene": "UniProtKB:Q9NQ34",
  "gene_name": "Transmembrane protein 9B"
}